{
  "term_label": "Unknown molecular function",
  "gene": "UniProtKB:Q8N715",
  "gene_symbol": "CCDC185",
  "gene_name": "Coiled-coil domain-containing protein 185",
  "term_id": "UNKNOWN:0001"
}